{
  "term_label": "cell-cell adhesion mediator activity",
  "gene_symbol": "LRRC4",
  "gene_name": "Leucine-rich repeat-containing protein 4",
  "term_id": "GO:0098632",
  "gene": "UniProtKB:Q9HBW1"
}